{
  "gene_symbol": "GDPGP1",
  "gene": "UniProtKB:Q6ZNW5",
  "term_label": "cytoplasm",
  "term_id": "GO:0005737",
  "gene_name": "GDP-D-glucose phosphorylase 1"
}